{
  "term_label": "plasma membrane tubulation",
  "gene": "UniProtKB:Q96RF0",
  "term_id": "GO:0097320",
  "gene_symbol": "SNX18",
  "gene_name": "Sorting nexin-18"
}